{
  "term_id": "UNKNOWN:0001",
  "gene": "UniProtKB:Q9BRU2",
  "term_label": "Unknown molecular function",
  "gene_symbol": "TCEAL7",
  "gene_name": "Transcription elongation factor A protein-like 7"
}